abieta-7,13-dien-18-al (NAD+) dehydrogenase activity [GO:0036188] (molecular function) Also known as: abieta-7,13-dien-18-al dehydrogenase activity, abietadienal dehydrogenase Sources: EC:1.2.1.74 Relationships: is a type of aldehyde dehydrogenase (NAD+) activity [GO:0004029] Definition: Catalysis of the reaction: abieta-7,13-diene-18-al + H2O + NAD+ = abieta-7,13-diene-18-oate + NADH + H+.